{
  "gene": "UniProtKB:Q16637",
  "gene_symbol": "SMN2",
  "term_label": "RNA binding",
  "term_id": "GO:0003723",
  "gene_name": "Survival motor neuron protein"
}